D-amino acid biosynthetic process [GO:0046437] (biological process) Also known as: D-amino acid anabolism, D-amino acid biosynthesis, D-amino acid formation, D-amino acid synthesis Subtypes: D-alanine biosynthetic process [GO:0030632], GO:0070179, GO:1900833 Sources: GOC:ai, GOC:jsg Relationships: is_a D-amino acid metabolic process [GO:0046416]; is_a non-proteinogenic amino acid biosynthetic process [GO:0170043]; is a type of alpha-amino acid biosynthetic process [GO:1901607] Definition: The chemical reactions and pathways resulting in the formation of D-amino acids, the D-enantiomers of amino acids.